RNA processing [GO:0006396] (biological process) Relationships: is a type of primary metabolic process [GO:0044238]; is part of gene expression [GO:0010467]; is part of GO:0032774 Sources: GOC:mah Subtypes: tRNA-type intron splice site recognition and cleavage [GO:0000379], mitochondrial RNA processing [GO:0000963], GO:0000966, rRNA processing [GO:0006364], GO:0006397, tRNA processing [GO:0008033], GO:0008380, snRNA processing [GO:0016180], RNA 3'-end processing [GO:0031123], chloroplast RNA processing [GO:0031425], sno(s)RNA processing [GO:0043144], regulatory ncRNA processing [GO:0070918], RNA polyadenylation at postsynapse [GO:0140235], GO:0141217, GO:0180035 Definition: Any process involved in the conversion of one or more primary RNA transcripts into one or more mature RNA molecules.